{
  "gene_symbol": "HSPA8",
  "gene": "UniProtKB:P11142",
  "term_label": "clathrin coat disassembly",
  "gene_name": "Heat shock cognate 71 kDa protein",
  "term_id": "GO:0072318"
}